ansamycin biosynthetic process [GO:0033070] (biological process) Relationships: is a type of polyketide biosynthetic process [GO:0030639]; is a type of lactam biosynthetic process [GO:0072339] Definition: The chemical reactions and pathways leading to the formation of ansamycins, any of a group of complex macrolactam compounds characterized by a cyclic structure in which an aliphatic ansa chain forms a bridge between two non-adjacent positions of a cyclic p-system; many exhibit antibacterial, antifungal or antitumor activity. Also known as: ansamycin anabolism, ansamycin biosynthesis, ansamycin formation, ansamycin synthesis Sources: GOC:mah, https://doi.org/10.1016/j.crci.2008.07.003